{
  "gene_name": "Inactive N-acetylated-alpha-linked acidic dipeptidase-like protein 2",
  "term_id": "UNKNOWN:0003",
  "gene": "UniProtKB:Q58DX5",
  "gene_symbol": "NAALADL2",
  "term_label": "Unknown cellular component"
}